phytoalexin metabolic process [GO:0052314] (biological process) Sources: Wikipedia:Phytoalexin Subtypes: GO:0052315, phytoalexin catabolic process [GO:0052316] Definition: The chemical reactions and pathways involving phytoalexins, any of a range of substances produced by plants as part of their defense response. Relationships: is a type of toxin metabolic process [GO:0009404] Also known as: phytoalexin metabolism